P-type cobalt transporter activity [GO:0032778] (molecular function) Also known as: ATP-dependent cobalt transmembrane transporter activity, ATPase-coupled cobalt transmembrane transporter activity, cobalt porter activity, cobalt transporting ATPase activity, cobalt-transporting ATPase activity Definition: Enables the transfer of a solute or solutes from one side of a membrane to the other according to the reaction: ATP + H2O + Co2+(out) = ADP + phosphate + Co2+(in). Relationships: is a type of cobalt ion transmembrane transporter activity [GO:0015087]; is a type of GO:0015662; is a type of GO:0019829 Sources: GOC:mlg, GOC:mtg_transport, ISBN:0815340729